{
  "term_id": "GO:0070588",
  "gene_name": "Sarcoplasmic_endoplasmic reticulum calcium ATPase 2",
  "gene_symbol": "ATP2A2",
  "gene": "UniProtKB:P16615",
  "term_label": "calcium ion transmembrane transport"
}